{
  "gene": "UniProtKB:Q8NE18",
  "gene_name": "Putative methyltransferase NSUN7",
  "term_label": "Unknown molecular function",
  "term_id": "UNKNOWN:0001",
  "gene_symbol": "NSUN7"
}